{
  "gene": "UniProtKB:O75179",
  "term_label": "Unknown molecular function",
  "term_id": "UNKNOWN:0001",
  "gene_symbol": "ANKRD17",
  "gene_name": "Ankyrin repeat domain-containing protein 17"
}